{
  "term_id": "GO:0061564",
  "gene_symbol": "SLC25A46",
  "gene": "UniProtKB:Q96AG3",
  "gene_name": "Mitochondrial outer membrane protein SLC25A46",
  "term_label": "axon development"
}